{
  "term_id": "UNKNOWN:0003",
  "term_label": "Unknown cellular component",
  "gene_symbol": "PRR33",
  "gene_name": "Proline-rich protein 33",
  "gene": "UniProtKB:A8MZF0"
}